{
  "gene": "UniProtKB:P54252",
  "term_id": "GO:0005634",
  "gene_name": "Ataxin-3",
  "gene_symbol": "ATXN3",
  "term_label": "nucleus"
}